regulation of tube size, open tracheal system [GO:0035151] (biological process) Relationships: is a type of regulation of tube size [GO:0035150]; is a type of regulation of tube architecture, open tracheal system [GO:0035152] Also known as: regulation of tracheal tube size References: PMID:10887083, PMID:12930776, PMID:12973360 Sources: GOC:mtg_sensu Definition: Ensuring that an epithelial tube in an open tracheal system is of the correct length and diameter. Tracheal tubes undergo highly regulated tube-size increases during development, expanding up to 40 times their initial size by the end of larval life. Tube size appears to be controlled by regulation of apical membrane expansion and secretion, rather than by changes in cell number, size or shape. Subtypes: regulation of tube diameter, open tracheal system [GO:0035158], regulation of tube length, open tracheal system [GO:0035159]